{
  "term_label": "Roundabout binding",
  "term_id": "GO:0048495",
  "gene_symbol": "SLIT2",
  "gene_name": "Slit homolog 2 protein",
  "gene": "UniProtKB:O94813"
}